negative regulation of somatic stem cell division [GO:1904676] (biological process) Definition: Any process that stops, prevents or reduces the frequency, rate or extent of somatic stem cell division. Relationships: is a type of negative regulation of cell division [GO:0051782]; is a type of regulation of somatic stem cell division [GO:1904675]; negatively regulates somatic stem cell division [GO:0048103] References: PMID:19409607 Sources: GOC:BHF, GOC:BHF_miRNA, GOC:TermGenie, GOC:rph, GO_REF:0000058 Also known as: down regulation of somatic stem cell division, down regulation of somatic stem cell renewal, down-regulation of somatic stem cell division, down-regulation of somatic stem cell renewal, downregulation of somatic stem cell division, downregulation of somatic stem cell renewal, negative regulation of somatic stem cell renewal, inhibition of somatic stem cell division, inhibition of somatic stem cell renewal